{
  "gene_symbol": "A1BG",
  "term_label": "transmembrane signaling receptor activity",
  "gene": "UniProtKB:P04217",
  "term_id": "GO:0004888",
  "gene_name": "Alpha-1B-glycoprotein"
}